positive regulation of translational initiation [GO:0045948] (biological process) Also known as: up regulation of translational initiation, up-regulation of translational initiation, upregulation of translational initiation, activation of translational initiation, stimulation of translational initiation Sources: GOC:go_curators Relationships: is a type of GO:0006446; is a type of GO:0045727; positively regulates translational initiation [GO:0006413] Definition: Any process that activates or increases the frequency, rate or extent of translational initiation. Subtypes: GO:0032058, positive regulation of translational initiation by iron [GO:0045994], GO:0070134, positive regulation of cytoplasmic translational initiation [GO:1904690]